{
  "term_id": "GO:0097730",
  "term_label": "non-motile cilium",
  "gene_name": "ADP-ribosylation factor-like protein 13A",
  "gene_symbol": "ARL13A",
  "gene": "UniProtKB:Q5H913"
}